tRNA-uridine aminocarboxypropyltransferase activity [GO:0016432] (MF) Definition: Catalysis of the reaction: a uridine in tRNA + S-adenosyl-L-methionine = a 3-[(3S)-3-amino-3-carboxypropyl]uridine in tRNA + S-methyl-5'-thioadenosine + H+. Sources: RHEA:62432 Also known as: S-adenosyl-L-methionine:tRNA-uridine 3-(3-amino-3-carboxypropyl)transferase activity Relationships: is a type of GO:0016765; is a type of catalytic activity, acting on a tRNA [GO:0140101]